{
  "gene_symbol": "WASHC5",
  "term_label": "actin filament polymerization",
  "term_id": "GO:0030041",
  "gene_name": "WASH complex subunit 5",
  "gene": "UniProtKB:Q12768"
}